{
  "gene_name": "RNA-binding motif, single-stranded-interacting protein 2",
  "term_label": "Unknown biological process",
  "gene": "UniProtKB:Q15434",
  "term_id": "UNKNOWN:0002",
  "gene_symbol": "RBMS2"
}